{
  "gene_name": "E3 SUMO-protein ligase PIAS4",
  "term_label": "regulation of transcription by RNA polymerase II",
  "term_id": "GO:0006357",
  "gene_symbol": "PIAS4",
  "gene": "UniProtKB:Q8N2W9"
}